{
  "gene_name": "Zinc finger protein 416",
  "term_label": "regulation of transcription by RNA polymerase II",
  "term_id": "GO:0006357",
  "gene_symbol": "ZNF416",
  "gene": "UniProtKB:Q9BWM5"
}